{
  "gene": "UniProtKB:P43308",
  "gene_symbol": "SSR2",
  "term_id": "UNKNOWN:0001",
  "gene_name": "Translocon-associated protein subunit beta",
  "term_label": "Unknown molecular function"
}